atrioventricular valve formation [GO:0003190] (BP) Sources: GOC:mtg_heart Subtypes: GO:0003192, tricuspid valve formation [GO:0003195] Relationships: is a type of GO:0003188; is part of atrioventricular valve morphogenesis [GO:0003181] Also known as: AV valve formation Definition: The developmental process pertaining to the initial formation of the atrioventricular valve from unspecified parts. This process begins with the specific processes that contribute to the appearance of the discrete structure and ends when the structural rudiment is recognizable.